{
  "gene_name": "Zinc finger protein 517",
  "gene_symbol": "ZNF517",
  "gene": "UniProtKB:Q6ZMY9",
  "term_id": "GO:0005634",
  "term_label": "nucleus"
}